positive regulation of growth [GO:0045927] (biological process) Also known as: up regulation of growth, up-regulation of growth, upregulation of growth, activation of growth, stimulation of growth Definition: Any process that activates or increases the rate or extent of growth, the increase in size or mass of all or part of an organism. Relationships: is a type of regulation of growth [GO:0040008]; is a type of GO:0048518; positively regulates growth [GO:0040007] Sources: GOC:go_curators Subtypes: positive regulation of cell growth [GO:0030307], positive regulation of growth rate [GO:0040010], positive regulation of developmental growth [GO:0048639], GO:0090033, positive regulation of secondary growth [GO:2000605]